{
  "gene_symbol": "MTR",
  "term_id": "GO:0050667",
  "term_label": "homocysteine metabolic process",
  "gene": "UniProtKB:Q99707",
  "gene_name": "Methionine synthase"
}